positive regulation of shade avoidance [GO:1902448] (biological process) Definition: Any process that activates or increases the frequency, rate or extent of shade avoidance. References: PMID:23763263 Sources: GOC:TermGenie Also known as: up regulation of shade avoidance, up-regulation of shade avoidance, upregulation of shade avoidance, activation of shade avoidance Relationships: is a type of GO:0048584; is a type of GO:1902446; positively regulates shade avoidance [GO:0009641]